{
  "gene": "UniProtKB:Q96PQ0",
  "term_id": "GO:0016020",
  "gene_symbol": "SORCS2",
  "gene_name": "VPS10 domain-containing receptor SorCS2",
  "term_label": "membrane"
}